xanthine dehydrogenase activity [GO:0004854] (molecular function) Relationships: is a type of oxidoreductase activity, acting on CH or CH2 groups, NAD or NADP as acceptor [GO:0016726] Sources: EC:1.17.1.4 Definition: Catalysis of the reaction: xanthine + NAD+ + H2O = urate + NADH + H+. Also known as: xanthine oxidoreductase activity, NAD-xanthine dehydrogenase activity, xanthine-NAD oxidoreductase activity, xanthine/NAD(+) oxidoreductase activity, xanthine/NAD+ oxidoreductase activity, xanthine:NAD+ oxidoreductase activity